{
  "gene": "UniProtKB:A0A1B0GVH7",
  "gene_symbol": "IQCM",
  "term_id": "UNKNOWN:0002",
  "gene_name": "IQ domain-containing protein M",
  "term_label": "Unknown biological process"
}